{
  "gene_name": "EKC_KEOPS complex subunit TP53RK",
  "term_label": "protein serine/threonine kinase activity",
  "gene_symbol": "TP53RK",
  "gene": "UniProtKB:Q96S44",
  "term_id": "GO:0004674"
}